{
  "gene_name": "Keratin, type II cuticular Hb2",
  "gene_symbol": "KRT82",
  "gene": "UniProtKB:Q9NSB4",
  "term_id": "GO:0045109",
  "term_label": "intermediate filament organization"
}